{
  "gene_name": "Kelch-like protein 41",
  "gene_symbol": "KLHL41",
  "term_id": "GO:0005737",
  "gene": "UniProtKB:O60662",
  "term_label": "cytoplasm"
}